{
  "term_id": "GO:0035556",
  "gene": "UniProtKB:Q96DD0",
  "gene_name": "Leucine-rich repeat-containing protein 39",
  "gene_symbol": "LRRC39",
  "term_label": "intracellular signal transduction"
}